quaternary ammonium group transmembrane transporter activity [GO:0015651] (MF) Definition: Enables the transfer of quaternary ammonium groups from one side of a membrane to the other. Quaternary ammonium groups are any compound that can be regarded as derived from ammonium hydroxide or an ammonium salt by replacement of all four hydrogen atoms of the NH4+ ion by organic groups. Sources: ISBN:0198506732 Relationships: is a type of transmembrane transporter activity [GO:0022857]; BFO_0000050 quaternary ammonium group transport [GO:0015697] Also known as: quaternary amine transmembrane transporter activity, quaternary ammonium compound transporter activity Subtypes: amino-acid betaine transmembrane transporter activity [GO:0015199], carnitine transmembrane transporter activity [GO:0015226], O-acyl-L-carnitine transmembrane transporter activity [GO:0015227], GO:0015418, quaternary ammonium group:proton symporter activity [GO:0015652], ATPase-coupled hydroxyectoine transmembrane transporter activity [GO:0033288], N-methylnicotinate transmembrane transporter activity [GO:0090417], thiamine pyrophosphate transmembrane transporter activity [GO:0090422], 4-(trimethylammonio)butanoate transmembrane transporter activity [GO:1901236]